{
  "gene_name": "Olfactory receptor 11L1",
  "term_id": "UNKNOWN:0003",
  "gene": "UniProtKB:Q8NGX0",
  "term_label": "Unknown cellular component",
  "gene_symbol": "OR11L1"
}